{
  "gene": "UniProtKB:P78316",
  "gene_symbol": "NOP14",
  "term_label": "nucleolus",
  "term_id": "GO:0005730",
  "gene_name": "Nucleolar protein 14"
}